tricarboxylic acid transport [GO:0006842] (biological process) Definition: The directed movement of tricarboxylic acids into, out of or within a cell, or between cells, by means of some agent such as a transporter or pore. Sources: GOC:krc Relationships: is a type of carboxylic acid transport [GO:0046942] Subtypes: citrate transport [GO:0015746], GO:0019271